{
  "gene": "UniProtKB:Q17RN3",
  "term_label": "tRNA-splicing ligase complex",
  "term_id": "GO:0072669",
  "gene_symbol": "FAM98C",
  "gene_name": "Protein FAM98C"
}